{
  "gene_name": "DnaJ homolog subfamily C member 5B",
  "gene_symbol": "DNAJC5B",
  "term_label": "Unknown cellular component",
  "gene": "UniProtKB:Q9UF47",
  "term_id": "UNKNOWN:0003"
}